{
  "term_id": "GO:0000978",
  "gene": "UniProtKB:Q9BYN7",
  "term_label": "RNA polymerase II cis-regulatory region sequence-specific DNA binding",
  "gene_name": "Zinc finger protein 341",
  "gene_symbol": "ZNF341"
}